integrin-mediated signaling pathway [GO:0007229] (biological process) Definition: The series of molecular signals initiated by an extracellular ligand binding to an integrin on the surface of a target cell, and ending with the regulation of a downstream cellular process, e.g. transcription. Regulation: regulated by regulation of integrin-mediated signaling pathway [GO:2001044]; negatively regulated by negative regulation of integrin-mediated signaling pathway [GO:2001045]; positively regulated by positive regulation of integrin-mediated signaling pathway [GO:2001046] Sources: GOC:mah, GOC:signaling Also known as: integrin-mediated signalling pathway Relationships: is_a cell surface receptor signaling pathway [GO:0007166]